{
  "gene": "UniProtKB:Q8TF17",
  "gene_name": "SH3 domain and tetratricopeptide repeat-containing protein 2",
  "term_label": "Unknown molecular function",
  "gene_symbol": "SH3TC2",
  "term_id": "UNKNOWN:0001"
}